{
  "gene": "UniProtKB:Q6ZVX7",
  "term_label": "SCF-dependent proteasomal ubiquitin-dependent protein catabolic process",
  "gene_name": "F-box only protein 50",
  "gene_symbol": "NCCRP1",
  "term_id": "GO:0031146"
}